nitrogenase (flavodoxin) activity [GO:0050142] (molecular function) Also known as: reduced flavodoxin:dinitrogen oxidoreductase (ATP-hydrolysing) Sources: EC:1.19.6.1, MetaCyc:NITROGENASE-FLAVODOXIN-RXN Relationships: is a type of oxidoreductase activity, acting on reduced flavodoxin as donor, dinitrogen as acceptor [GO:0016738]; is part of nitrogen fixation [GO:0009399] Definition: Catalysis of the reaction: 6 reduced flavodoxin + 6 H+ + N2 + n ATP = 6 oxidized flavodoxin + 2 NH3 + n ADP + n phosphate.